{
  "term_label": "cell surface receptor signaling pathway",
  "gene": "UniProtKB:Q6UY13",
  "term_id": "GO:0007166",
  "gene_name": "Putative uncharacterized protein UNQ5830_PRO19650_PRO19816",
  "gene_symbol": "UNQ5830/PRO19650/PRO19816"
}